{
  "gene_symbol": "NPIPA7",
  "term_label": "Unknown cellular component",
  "gene": "UniProtKB:E9PJI5",
  "term_id": "UNKNOWN:0003",
  "gene_name": "Nuclear pore complex-interacting protein family member A7"
}